{
  "term_id": "GO:0036435",
  "term_label": "K48-linked polyubiquitin modification-dependent protein binding",
  "gene": "UniProtKB:Q04323",
  "gene_symbol": "UBXN1",
  "gene_name": "UBX domain-containing protein 1"
}